{
  "gene": "UniProtKB:P02671",
  "term_label": "protein-macromolecule adaptor activity",
  "term_id": "GO:0030674",
  "gene_name": "Fibrinogen alpha chain",
  "gene_symbol": "FGA"
}